stem cell development [GO:0048864] (biological process) Subtypes: neural crest cell development [GO:0014032] Relationships: is a type of cell development [GO:0048468]; BFO_0000050 stem cell differentiation [GO:0048863] Definition: The process whose specific outcome is the progression of the stem cell over time, from its formation to the mature structure. Cell development does not include the steps involved in committing a cell to its specific fate. Sources: CL:0000034, GOC:isa_complete